{
  "gene_name": "T cell receptor delta constant",
  "gene": "UniProtKB:B7Z8K6",
  "term_id": "UNKNOWN:0003",
  "gene_symbol": "TRDC",
  "term_label": "Unknown cellular component"
}